ceramide metabolic process [GO:0006672] (biological process) Definition: The chemical reactions and pathways involving ceramides, any N-acylated sphingoid. Subtypes: ganglioside metabolic process [GO:0001573], glycosylceramide metabolic process [GO:0006677], ceramide biosynthetic process [GO:0046513], GO:0046514 Relationships: is a type of sphingolipid metabolic process [GO:0006665]; is a type of GO:0043603 Sources: ISBN:0198547684 Also known as: ceramide metabolism